{
  "gene": "UniProtKB:P0DPF2",
  "term_id": "UNKNOWN:0002",
  "gene_name": "Neuroblastoma breakpoint family member 20",
  "term_label": "Unknown biological process",
  "gene_symbol": "NBPF20"
}